{
  "gene_symbol": "OSCAR",
  "gene_name": "Osteoclast-associated immunoglobulin-like receptor",
  "gene": "UniProtKB:Q8IYS5",
  "term_id": "GO:0030316",
  "term_label": "osteoclast differentiation"
}